{
  "term_label": "Unknown cellular component",
  "gene_symbol": "HCFC1R1",
  "term_id": "UNKNOWN:0003",
  "gene_name": "Host cell factor C1 regulator 1",
  "gene": "UniProtKB:Q9NWW0"
}